{
  "term_id": "GO:0004622",
  "gene_symbol": "PNPLA6",
  "gene_name": "Patatin-like phospholipase domain-containing protein 6",
  "term_label": "phosphatidylcholine lysophospholipase activity",
  "gene": "UniProtKB:Q8IY17"
}